{
  "gene_name": "RIMS-binding protein 3A",
  "term_id": "GO:0030156",
  "gene_symbol": "RIMBP3",
  "gene": "UniProtKB:Q9UFD9",
  "term_label": "benzodiazepine receptor binding"
}